{
  "gene_symbol": "VWA2",
  "term_id": "GO:0005615",
  "gene": "UniProtKB:Q5GFL6",
  "term_label": "extracellular space",
  "gene_name": "von Willebrand factor A domain-containing protein 2"
}